{
  "gene": "UniProtKB:Q8WZA6",
  "term_label": "plasma membrane",
  "gene_name": "Olfactory receptor 1E3",
  "gene_symbol": "OR1E3",
  "term_id": "GO:0005886"
}